{
  "gene_name": "Bromodomain and WD repeat-containing protein 1",
  "term_label": "nucleus",
  "gene_symbol": "BRWD1",
  "term_id": "GO:0005634",
  "gene": "UniProtKB:Q9NSI6"
}